{
  "term_label": "Unknown molecular function",
  "term_id": "UNKNOWN:0001",
  "gene": "UniProtKB:Q9NU53",
  "gene_name": "Glycoprotein integral membrane protein 1",
  "gene_symbol": "GINM1"
}